{
  "term_id": "UNKNOWN:0003",
  "term_label": "Unknown cellular component",
  "gene_symbol": "ADO",
  "gene": "UniProtKB:Q96SZ5",
  "gene_name": "2-aminoethanethiol dioxygenase"
}